{
  "gene_name": "Calcium_calmodulin-dependent protein kinase II inhibitor 2",
  "term_id": "UNKNOWN:0003",
  "gene_symbol": "CAMK2N2",
  "term_label": "Unknown cellular component",
  "gene": "UniProtKB:Q96S95"
}